2-methylguanosine metabolic process [GO:0080180] (biological process) Definition: The chemical reactions and pathways involving 2-methylguanosine. Sources: GOC:tb Relationships: is a type of purine ribonucleoside metabolic process [GO:0046128]